{
  "gene_name": "Epidermal growth factor receptor kinase substrate 8-like protein 2",
  "gene": "UniProtKB:Q9H6S3",
  "term_label": "regulation of Rho protein signal transduction",
  "term_id": "GO:0035023",
  "gene_symbol": "EPS8L2"
}